{
  "gene_name": "Protein Wnt-2",
  "term_id": "GO:0005109",
  "gene": "UniProtKB:P09544",
  "term_label": "frizzled binding",
  "gene_symbol": "WNT2"
}